{
  "term_id": "GO:0005254",
  "term_label": "chloride channel activity",
  "gene_symbol": "GABRG3",
  "gene_name": "Gamma-aminobutyric acid receptor subunit gamma-3",
  "gene": "UniProtKB:Q99928"
}